protein localization to endoplasmic reticulum exit site [GO:0070973] (biological process) Sources: GOC:mah Also known as: protein localisation to endoplasmic reticulum exit site, protein localization to ER exit site Relationships: is_a protein localization to endoplasmic reticulum [GO:0070972] Definition: A process in which a protein is transported to, or maintained in, a location at an endoplasmic reticulum exit site.